{
  "term_label": "interkinetic nuclear migration",
  "gene": "UniProtKB:Q8N960",
  "gene_symbol": "CEP120",
  "term_id": "GO:0022027",
  "gene_name": "Centrosomal protein of 120 kDa"
}